tRNA queuosine(34) biosynthetic process [GO:0008616] (biological process) Subtypes: de novo tRNA queuosine(34) biosynthetic process [GO:0160253], GO:0160254, tRNA queuosine(34) biosynthetic process from salvaged queuine [GO:0160255] Relationships: is a type of tRNA wobble guanine modification [GO:0002099]; is a type of biosynthetic process [GO:0009058] Also known as: queuosine anabolism, queuosine biosynthesis, queuosine biosynthetic process, queuosine formation, queuosine synthesis Definition: The chemical reactions and pathways resulting in the formation of queuosines, a series of nucleosides found in position 34 of tRNA and having an additional pentenyl ring added via an NH group to the methyl group of 7-methylguanosine. The pentenyl ring may carry other substituents. The wobble nucleoside of the tRNA sequence  (position 34) corresponds to the first position of the anticodon. References: PMID:28208705, PMID:39600051